dorsal/ventral axis specification, ovarian follicular epithelium [GO:0008069] (biological process) Sources: GOC:bf, GOC:dph, GOC:mtg_sensu, GOC:tb Definition: Polarization of the ovarian follicle cells along the dorsal/ventral axis. An example of this process is found in Drosophila melanogaster. Also known as: dorsal-ventral axis specification, ovarian follicular epithelium, dorsal/ventral axis determination, ovarian follicular epithelium, dorsoventral axis specification, ovarian follicular epithelium, dorsal/ventral axis determination, follicular epithelium Subtypes: GO:0008070, maternal determination of dorsal/ventral axis, ovarian follicular epithelium, soma encoded [GO:0008071] Relationships: is a type of developmental process involved in reproduction [GO:0003006]; is a type of dorsal/ventral axis specification [GO:0009950]; is a type of establishment or maintenance of polarity of follicular epithelium [GO:0016334]; is part of GO:0030707